regulation of salivary gland boundary specification [GO:0045704] (biological process) Also known as: regulation of salivary gland determination Relationships: is a type of regulation of developmental process [GO:0050793]; is a type of regulation of multicellular organismal process [GO:0051239]; regulates GO:0007432 Sources: GOC:go_curators, GOC:tb Definition: Any process that modulates the frequency, rate or extent of salivary gland determination. Subtypes: negative regulation of salivary gland boundary specification [GO:0045705], GO:0045706, regulation of adult salivary gland boundary specification [GO:0045707], regulation of larval salivary gland boundary specification [GO:0045708]